{
  "gene": "UniProtKB:O95998",
  "term_id": "GO:0042007",
  "gene_name": "Interleukin-18-binding protein",
  "term_label": "interleukin-18 binding",
  "gene_symbol": "IL18BP"
}